oxalate transport [GO:0019532] (biological process) Also known as: ethanedioate transport, ethanedioic acid transport, oxalic acid transport Relationships: is a type of dicarboxylic acid transport [GO:0006835] Subtypes: GO:0046724 Definition: The directed movement of oxalate into, out of or within a cell, or between cells, by means of some agent such as a transporter or pore. Oxalate, or ethanedioic acid, occurs in many plants and is highly toxic to animals. Sources: ISBN:0198506732